regulation of viral translation [GO:1904971] (biological process) Also known as: regulation of viral protein anabolism, regulation of viral protein biosynthesis, regulation of viral protein biosynthetic process, regulation of viral protein formation, regulation of viral protein synthesis Relationships: is a type of regulation of viral process [GO:0050792]; regulates GO:0019081 References: PMID:19666601 Sources: GOC:TermGenie, GOC:bhm, GO_REF:0000058 Subtypes: negative regulation of viral translation [GO:1904972], positive regulation of viral translation [GO:1904973] Definition: Any process that modulates the frequency, rate or extent of viral translation.